regulation of reactive oxygen species biosynthetic process [GO:1903426] (biological process) Relationships: is a type of regulation of biosynthetic process [GO:0009889]; is a type of regulation of reactive oxygen species metabolic process [GO:2000377]; regulates GO:1903409 References: PMID:24252804 Sources: GOC:PARL, GOC:TermGenie, GOC:bf, GO_REF:0000058 Subtypes: regulation of hydrogen peroxide biosynthetic process [GO:0010728], negative regulation of reactive oxygen species biosynthetic process [GO:1903427], positive regulation of reactive oxygen species biosynthetic process [GO:1903428] Also known as: regulation of reactive oxygen species anabolism, regulation of reactive oxygen species biosynthesis, regulation of reactive oxygen species formation, regulation of reactive oxygen species synthesis, regulation of ROS formation, regulation of ROS generation, regulation of reactive oxygen species generation Definition: Any process that modulates the frequency, rate or extent of reactive oxygen species biosynthetic process.